{
  "term_label": "extracellular space",
  "gene_symbol": "NMB",
  "term_id": "GO:0005615",
  "gene_name": "Neuromedin-B",
  "gene": "UniProtKB:P08949"
}